hydroxymalonate dehydrogenase activity [GO:0047993] (molecular function) Definition: Catalysis of the reaction: hydroxymalonate + NAD+ = H+ + NADH + oxomalonate. Sources: EC:1.1.1.167, RHEA:11284 Relationships: is a type of GO:0016616 Also known as: hydroxymalonate:NAD+ oxidoreductase activity